{
  "term_label": "cytoplasmic vesicle",
  "gene_name": "Flotillin-1",
  "gene_symbol": "FLOT1",
  "term_id": "GO:0031410",
  "gene": "UniProtKB:O75955"
}